cytidine transmembrane transporter activity [GO:0015212] (molecular function) Definition: Enables the transfer of cytidine, cytosine riboside, from one side of a membrane to the other. Sources: GOC:go_curators Relationships: is a type of pyrimidine nucleoside transmembrane transporter activity [GO:0015214]; is part of cytidine transport [GO:0015861]